{
  "gene_symbol": "MKX",
  "term_id": "GO:0005634",
  "gene": "UniProtKB:Q8IYA7",
  "gene_name": "Homeobox protein Mohawk",
  "term_label": "nucleus"
}